{
  "gene_symbol": "GPR4",
  "gene": "UniProtKB:P46093",
  "term_id": "GO:0004930",
  "term_label": "G protein-coupled receptor activity",
  "gene_name": "G-protein coupled receptor 4"
}